{
  "term_label": "phosphatidylcholine transporter activity",
  "gene_symbol": "PITPNB",
  "term_id": "GO:0008525",
  "gene_name": "Phosphatidylinositol transfer protein beta isoform",
  "gene": "UniProtKB:P48739"
}